{
  "term_id": "GO:0071254",
  "gene_name": "U7 snRNA-associated Sm-like protein LSm10",
  "gene_symbol": "LSM10",
  "term_label": "cytoplasmic U snRNP body",
  "gene": "UniProtKB:Q969L4"
}